siderophore-iron import into cell [GO:0033214] (biological process) Definition: A process in which iron (Fe3+) is solubilized by ferric iron-specific chelators, known as siderophores is imported into the cell by transmembrane transport or endocytosis. Subtypes: ferric-enterobactin import into cell [GO:0015685], GO:0015686, GO:0015687 Relationships: is a type of import into cell [GO:0098657]; is a type of siderophore-dependent iron import pathway [GO:0180060]; is a type of iron coordination entity transport [GO:1901678]; has part iron ion import across plasma membrane [GO:0098711] Also known as: iron assimilation by chelation and transport References: PMID:16963626 Sources: GOC:vw